{
  "term_id": "UNKNOWN:0002",
  "gene": "UniProtKB:Q16655",
  "gene_name": "Melanoma antigen recognized by T-cells 1",
  "term_label": "Unknown biological process",
  "gene_symbol": "MLANA"
}